{
  "term_label": "negative regulation of transcription by RNA polymerase II",
  "gene": "UniProtKB:O75182",
  "term_id": "GO:0000122",
  "gene_name": "Paired amphipathic helix protein Sin3b",
  "gene_symbol": "SIN3B"
}